{
  "term_label": "developmental pigmentation",
  "gene_name": "Endothelin-1 receptor",
  "gene": "UniProtKB:P25101",
  "gene_symbol": "EDNRA",
  "term_id": "GO:0048066"
}